cytoskeleton-dependent intracellular transport [GO:0030705] (biological process) Sources: GOC:mah Definition: The directed movement of substances along cytoskeletal fibers such as microfilaments or microtubules within a cell. Subtypes: transport along microtubule [GO:0010970], cytoskeleton-dependent cytoplasmic transport, nurse cell to oocyte [GO:0019749], actin filament-based transport [GO:0099515], vesicle cytoskeletal trafficking [GO:0099518] Relationships: is a type of GO:0046907